peptidyl-cysteine methylation [GO:0018125] (biological process) Relationships: is a type of protein methylation [GO:0006479]; is a type of peptidyl-cysteine modification [GO:0018198] Sources: RESID:AA0234 Definition: The methylation of peptidyl-cysteine to form peptidyl-S-methyl-L-cysteine.